{
  "term_label": "RNA polymerase II cis-regulatory region sequence-specific DNA binding",
  "gene_name": "Homeobox protein EMX2",
  "term_id": "GO:0000978",
  "gene_symbol": "EMX2",
  "gene": "UniProtKB:Q04743"
}